Tec1p-Ste12p-Dig1p complex [GO:1990527] (cellular component) References: PMID:16782869 Sources: GOC:rb Relationships: is a type of protein-containing complex [GO:0032991] Definition: A multiprotein complex that is involved in the transcriptional regulation of primarily filamentation genes, but also mating genes, in the yeast S. cerevisiae.